{
  "term_label": "mitochondrial citrate transmembrane transport",
  "gene_symbol": "SLC25A1",
  "term_id": "GO:0006843",
  "gene_name": "Tricarboxylate transport protein, mitochondrial",
  "gene": "UniProtKB:P53007"
}